{
  "gene_name": "Epithelial cell adhesion molecule",
  "term_id": "UNKNOWN:0002",
  "term_label": "Unknown biological process",
  "gene_symbol": "EPCAM",
  "gene": "UniProtKB:P16422"
}